{
  "gene_name": "Apolipoprotein C-II",
  "term_label": "phospholipase activator activity",
  "gene_symbol": "APOC2",
  "gene": "UniProtKB:P02655",
  "term_id": "GO:0016004"
}